{
  "gene_name": "Serine_threonine-protein kinase 4",
  "gene": "UniProtKB:Q13043",
  "gene_symbol": "STK4",
  "term_id": "GO:0043408",
  "term_label": "regulation of MAPK cascade"
}